regulation of Wnt signaling pathway involved in heart development [GO:0003307] (biological process) Definition: Any process that modulates the rate, frequency, or extent of the series of molecular signals initiated by binding of Wnt protein to a frizzled family receptor on the surface of the target cell, resulting a change in cell state that contributes to the progression of the heart over time. Sources: GOC:mtg_heart Also known as: regulation of Wnt receptor signaling pathway involved in heart development, regulation of Wnt receptor signalling pathway involved in heart development, regulation of Wnt-activated signaling pathway involved in heart development Relationships: is a type of regulation of Wnt signaling pathway [GO:0030111]; regulates Wnt signaling pathway involved in heart development [GO:0003306] Subtypes: negative regulation of Wnt signaling pathway involved in heart development [GO:0003308]